{
  "gene_name": "Myosin regulatory light chain 12A",
  "gene_symbol": "MYL12A",
  "term_label": "Unknown biological process",
  "term_id": "UNKNOWN:0002",
  "gene": "UniProtKB:P19105"
}